negative regulation of insulin receptor signaling pathway [GO:0046627] (biological process) Definition: Any process that stops, prevents, or reduces the frequency, rate or extent of insulin receptor signaling. Sources: GOC:bf Also known as: down regulation of insulin receptor signaling pathway, down-regulation of insulin receptor signaling pathway, downregulation of insulin receptor signaling pathway, negative regulation of insulin receptor signalling pathway, inhibition of insulin receptor signaling pathway Relationships: is a type of negative regulation of signal transduction [GO:0009968]; is_a regulation of insulin receptor signaling pathway [GO:0046626]; is a type of GO:1900077; negatively regulates GO:0008286 Subtypes: negative regulation of insulin receptor signaling pathway by insulin receptor internalization [GO:0038014]